{
  "gene_symbol": "LRATD2",
  "term_label": "Unknown molecular function",
  "gene_name": "Protein LRATD2",
  "term_id": "UNKNOWN:0001",
  "gene": "UniProtKB:Q96KN1"
}